detection of carbon dioxide [GO:0003031] (biological process) Sources: GOC:mtg_cardio Relationships: is a type of detection of chemical stimulus [GO:0009593] Subtypes: detection of carbon dioxide by vasomotor center [GO:0002013], GO:0003021 Definition: The series of events in which a carbon dioxide stimulus is received by a cell and converted into a molecular signal.